{
  "term_id": "GO:0060538",
  "gene_symbol": "MYMX",
  "gene_name": "Protein myomixer",
  "gene": "UniProtKB:A0A1B0GTQ4",
  "term_label": "skeletal muscle organ development"
}